{
  "gene": "UniProtKB:Q13277",
  "term_label": "vesicle docking",
  "gene_symbol": "STX3",
  "term_id": "GO:0048278",
  "gene_name": "Syntaxin-3"
}